dolichyl-phosphate-mannose-protein mannosyltransferase Pmt1p-Pmt3p dimer complex [GO:0097583] (cellular component) Definition: A protein dimer complex that possesses dolichyl-phosphate-mannose-protein mannosyltransferase activity and, in S. cerevisiae, is composed of Pmt1p-Pmt3p. References: PMID:12551906 Sources: GOC:jd Also known as: Pmt1p-Pmt3p complex Relationships: is a type of GO:0031502